histone butyryltransferase activity [GO:0140069] (molecular function) Relationships: is a type of peptide butyryltransferase activity [GO:0140065]; is a type of histone modifying activity [GO:0140993] References: PMID:27105113 Definition: Catalysis of the reaction: butyryl-CoA + histone = CoA + butyryl-histone.